{
  "gene": "UniProtKB:Q9Y4E5",
  "gene_symbol": "ZNF451",
  "term_id": "GO:0003714",
  "term_label": "transcription corepressor activity",
  "gene_name": "E3 SUMO-protein ligase ZNF451"
}